{
  "gene_name": "Succinate--CoA ligase [ADP-forming] subunit beta, mitochondrial",
  "term_id": "GO:0006099",
  "term_label": "tricarboxylic acid cycle",
  "gene": "UniProtKB:Q9P2R7",
  "gene_symbol": "SUCLA2"
}